{
  "gene": "UniProtKB:P48745",
  "term_label": "extracellular matrix",
  "gene_name": "CCN family member 3",
  "term_id": "GO:0031012",
  "gene_symbol": "CCN3"
}